cytosylglucuronate decarboxylase activity [GO:1990965] (molecular function) Definition: Catalysis of the reaction: cytosylglucuronic acid + H+ = cytosylarabinopyranose + CO2. Relationships: is a type of carboxy-lyase activity [GO:0016831] Note: This enzymatic activity was shown to be involved in the bacterial blasticidin S biosynthetic pathway. References: PMID:23874663 Sources: GOC:pr, GOC:tb